{
  "gene_symbol": "AREL1",
  "term_id": "GO:0005829",
  "gene_name": "Apoptosis-resistant E3 ubiquitin protein ligase 1",
  "term_label": "cytosol",
  "gene": "UniProtKB:O15033"
}